{
  "gene_name": "Inositol-3-phosphate synthase 1",
  "gene_symbol": "ISYNA1",
  "gene": "UniProtKB:Q9NPH2",
  "term_label": "inositol-3-phosphate synthase activity",
  "term_id": "GO:0004512"
}